{
  "gene_name": "Programmed cell death protein 10",
  "term_id": "GO:0019901",
  "term_label": "protein kinase binding",
  "gene": "UniProtKB:Q9BUL8",
  "gene_symbol": "PDCD10"
}